{
  "gene_symbol": "SASH3",
  "gene": "UniProtKB:O75995",
  "term_label": "positive regulation of adaptive immune response",
  "gene_name": "SAM and SH3 domain-containing protein 3",
  "term_id": "GO:0002821"
}